ochratoxin A catabolic process [GO:1900817] (biological process) Definition: The chemical reactions and pathways resulting in the breakdown of ochratoxin A. Relationships: is_a modified amino acid catabolic process [GO:0042219]; is a type of amide metabolic process [GO:0043603]; is a type of monocarboxylic acid catabolic process [GO:0072329]; is a type of organohalogen metabolic process [GO:0090345]; is_a secondary metabolite catabolic process [GO:0090487] Sources: GOC:TermGenie, GOC:di Also known as: ochratoxin A breakdown, ochratoxin A catabolism, ochratoxin A degradation